{
  "gene": "UniProtKB:Q9P1Q0",
  "gene_symbol": "VPS54",
  "term_id": "GO:0006896",
  "term_label": "Golgi to vacuole transport",
  "gene_name": "Vacuolar protein sorting-associated protein 54"
}